{
  "term_id": "GO:0030010",
  "term_label": "establishment of cell polarity",
  "gene": "UniProtKB:Q8TEW8",
  "gene_name": "Partitioning defective 3 homolog B",
  "gene_symbol": "PARD3B"
}